{
  "gene_symbol": "SPATA9",
  "term_label": "Unknown cellular component",
  "term_id": "UNKNOWN:0003",
  "gene_name": "Spermatogenesis-associated protein 9",
  "gene": "UniProtKB:Q9BWV2"
}